{
  "gene_name": "Low-density lipoprotein receptor-related protein 5-like protein",
  "term_label": "Unknown cellular component",
  "term_id": "UNKNOWN:0003",
  "gene_symbol": "LRP5L",
  "gene": "UniProtKB:A4QPB2"
}